{
  "gene": "UniProtKB:A7KAX9",
  "term_id": "GO:0150052",
  "term_label": "regulation of postsynapse assembly",
  "gene_symbol": "ARHGAP32",
  "gene_name": "Rho GTPase-activating protein 32"
}